{
  "gene_symbol": "CENPE",
  "term_id": "GO:0005874",
  "gene_name": "Centromere-associated protein E",
  "gene": "UniProtKB:Q02224",
  "term_label": "microtubule"
}